amylin receptor 1 signaling pathway [GO:0150059] (biological process) References: PMID:22500019 Sources: GOC:aruk, GOC:bc Relationships: is a type of amylin receptor signaling pathway [GO:0097647] Also known as: AMY1 signaling pathway Definition: The series of molecular signals initiated by an extracellular amylin, or another ligand, combining with an amylin receptor 1 (AMY1), a G protein-coupled receptor complex, on the surface of the target cell. Other ligands that have been shown to initiate the AMY1 signaling pathway include the calcitonin related peptide (CGRP) and adrenomedullin (AM/ADM).